{
  "term_label": "extracellular region",
  "gene_symbol": "KNG1",
  "term_id": "GO:0005576",
  "gene": "UniProtKB:P01042",
  "gene_name": "Kininogen-1"
}